dAMP catabolic process [GO:0046059] (BP) Definition: The chemical reactions and pathways resulting in the breakdown of dAMP, deoxyadenosine monophosphate (2'-deoxyadenosine 5'-phosphate). Also known as: dAMP breakdown, dAMP catabolism, dAMP degradation Relationships: is a type of purine deoxyribonucleotide catabolic process [GO:0009155]; is a type of purine deoxyribonucleoside monophosphate catabolic process [GO:0009172]; is a type of dAMP metabolic process [GO:0046053] Sources: GOC:go_curators